{
  "term_label": "microtubule binding",
  "gene_name": "Disks large-associated protein 5",
  "gene_symbol": "DLGAP5",
  "gene": "UniProtKB:Q15398",
  "term_id": "GO:0008017"
}